sodium ion homeostasis [GO:0055078] (biological process) Sources: GOC:ai, GOC:jid, GOC:mah Subtypes: intracellular sodium ion homeostasis [GO:0006883] Definition: Any process involved in the maintenance of an internal steady state of sodium ions within an organism or cell. Relationships: is a type of monoatomic cation homeostasis [GO:0055080]; is_a inorganic ion homeostasis [GO:0098771]